{
  "term_id": "GO:0005654",
  "term_label": "nucleoplasm",
  "gene": "UniProtKB:Q5VZF2",
  "gene_symbol": "MBNL2",
  "gene_name": "Muscleblind-like protein 2"
}